salicylic acid metabolic process [GO:0009696] (biological process) Sources: ISBN:0943088399 Subtypes: GO:0009697, salicylic acid catabolic process [GO:0046244] Regulation: regulated by regulation of salicylic acid metabolic process [GO:0010337] Definition: The chemical reactions and pathways involving of salicylic acid (2-hydroxybenzoic acid), a derivative of benzoic acid. Also known as: salicylic acid metabolism Relationships: is_a phenol-containing compound metabolic process [GO:0018958]; is a type of monocarboxylic acid metabolic process [GO:0032787]; is a type of GO:0042537